TRAMP-dependent tRNA surveillance pathway [GO:0071038] (BP) Definition: A nuclear tRNA surveillance pathway, dependent on the TRAMP exosome adaptor and the nuclear exosome. Relationships: is a type of nuclear RNA surveillance [GO:0071027]; is a type of tRNA surveillance [GO:0106354] References: PMID:35901126 Sources: GOC:vw